{
  "gene_symbol": "COQ8B",
  "gene_name": "Atypical kinase COQ8B, mitochondrial",
  "term_label": "ubiquinone biosynthetic process",
  "term_id": "GO:0006744",
  "gene": "UniProtKB:Q96D53"
}